{
  "term_id": "GO:0005737",
  "gene": "UniProtKB:Q92945",
  "gene_symbol": "KHSRP",
  "term_label": "cytoplasm",
  "gene_name": "Far upstream element-binding protein 2"
}